{
  "gene": "UniProtKB:O60293",
  "gene_name": "Zinc finger C3H1 domain-containing protein",
  "gene_symbol": "ZFC3H1",
  "term_id": "UNKNOWN:0002",
  "term_label": "Unknown biological process"
}